{
  "gene_name": "CUGBP Elav-like family member 6",
  "gene": "UniProtKB:Q96J87",
  "term_id": "GO:0006376",
  "term_label": "mRNA splice site recognition",
  "gene_symbol": "CELF6"
}